{
  "term_id": "GO:0070776",
  "gene_name": "Bromodomain-containing protein 1",
  "gene": "UniProtKB:O95696",
  "term_label": "MOZ/MORF histone acetyltransferase complex",
  "gene_symbol": "BRD1"
}